glucuronidase activity [GO:0046574] (molecular function) Relationships: is a type of GO:0004553 Subtypes: beta-glucuronidase activity [GO:0004566], hyaluronoglucuronidase activity [GO:0033906], acyl-glucuronidase activity [GO:0036237], GO:0046559, glucuronosyl-disulfoglucosamine glucuronidase activity [GO:0047404], glycyrrhizinate beta-glucuronidase activity [GO:0047967], baicalin beta-D-glucuronidase activity [GO:0052748] References: PMID:10441389, PMID:12044176 Definition: Catalysis of the hydrolysis of glucuronosides, yielding free glucuronic acid. Also known as: glucuronyl hydrolase activity, glycuronidase activity